{
  "term_id": "GO:0004674",
  "gene": "UniProtKB:Q8WXR4",
  "gene_name": "Myosin-IIIb",
  "term_label": "protein serine/threonine kinase activity",
  "gene_symbol": "MYO3B"
}